{
  "term_id": "GO:0042393",
  "term_label": "histone binding",
  "gene_name": "Condensin complex subunit 1",
  "gene_symbol": "NCAPD2",
  "gene": "UniProtKB:Q15021"
}